{
  "gene_symbol": "CNOT3",
  "gene": "UniProtKB:O75175",
  "term_id": "GO:0000289",
  "term_label": "nuclear-transcribed mRNA poly(A) tail shortening",
  "gene_name": "CCR4-NOT transcription complex subunit 3"
}